{
  "gene_name": "Ribosome biogenesis protein NOP53",
  "gene_symbol": "NOP53",
  "gene": "UniProtKB:Q9NZM5",
  "term_id": "GO:0006364",
  "term_label": "rRNA processing"
}